{
  "term_label": "early endosome",
  "gene_name": "Ras-related protein Rab-5A",
  "gene": "UniProtKB:P20339",
  "term_id": "GO:0005769",
  "gene_symbol": "RAB5A"
}